{
  "term_label": "Unknown molecular function",
  "gene": "UniProtKB:Q6ICB0",
  "gene_symbol": "DESI1",
  "term_id": "UNKNOWN:0001",
  "gene_name": "Desumoylating isopeptidase 1"
}